ACF complex [GO:0016590] (cellular component) Also known as: ATP-utilizing chromatin assembly and remodeling factor complex References: PMID:12192034, PMID:15284901, PMID:16568949, PMID:21810179 Sources: GOC:bf, GOC:krc Definition: An ISWI complex that contains an ATPase subunit of the ISWI family (SNF2H in mammals, Isw2 in S. cerevisiae), an ACF1 homolog, and generally no other subunits, though Xenopus is an exception with a third non-conserved subunit. ACF plays roles in regulation of RNA polymerase II transcription and in DNA replication and repair. Relationships: is a type of ISWI-type complex [GO:0031010]